{
  "gene_name": "Regulating synaptic membrane exocytosis protein 1",
  "gene": "UniProtKB:Q86UR5",
  "term_label": "structural constituent of presynaptic active zone",
  "gene_symbol": "RIMS1",
  "term_id": "GO:0098882"
}